{
  "term_id": "UNKNOWN:0002",
  "gene": "UniProtKB:Q9HB19",
  "term_label": "Unknown biological process",
  "gene_name": "Pleckstrin homology domain-containing family A member 2",
  "gene_symbol": "PLEKHA2"
}